{
  "term_label": "regulation of transcription by RNA polymerase II",
  "gene": "UniProtKB:Q99453",
  "gene_name": "Paired mesoderm homeobox protein 2B",
  "gene_symbol": "PHOX2B",
  "term_id": "GO:0006357"
}